{
  "gene_name": "Neuromodulin",
  "term_id": "GO:0014069",
  "gene_symbol": "GAP43",
  "gene": "UniProtKB:P17677",
  "term_label": "postsynaptic density"
}